dense fibrillar component [GO:0001651] (cellular component) References: PMID:10754561 Definition: A structure found in the nucleolus, which contains newly synthesized preribosomal RNA (pre-rRNA) and a collection of proteins. Also known as: pars fibrosa Relationships: is a type of cellular anatomical structure [GO:0110165]; is part of GO:0005730